{
  "gene_symbol": "C16orf95",
  "term_label": "Unknown cellular component",
  "gene_name": "Uncharacterized protein C16orf95",
  "gene": "UniProtKB:Q9H693",
  "term_id": "UNKNOWN:0003"
}